{
  "gene_symbol": "LRP11",
  "gene_name": "Low-density lipoprotein receptor-related protein 11",
  "term_id": "UNKNOWN:0003",
  "term_label": "Unknown cellular component",
  "gene": "UniProtKB:Q86VZ4"
}